positive regulation of type IV hypersensitivity [GO:0001809] (BP) Also known as: up regulation of type IV hypersensitivity, up-regulation of type IV hypersensitivity, upregulation of type IV hypersensitivity, activation of type IV hypersensitivity, stimulation of type IV hypersensitivity Sources: GOC:add, ISBN:0781735149 Definition: Any process that activates or increases the frequency, rate or extent of type IV hypersensitivity, a type of inflammatory response. Relationships: is a type of regulation of type IV hypersensitivity [GO:0001807]; is a type of positive regulation of T cell mediated immunity [GO:0002711]; is a type of positive regulation of hypersensitivity [GO:0002885]; positively regulates type IV hypersensitivity [GO:0001806]